{
  "gene_name": "Zinc finger protein 14 homolog",
  "gene_symbol": "ZFP14",
  "gene": "UniProtKB:Q9HCL3",
  "term_label": "nucleus",
  "term_id": "GO:0005634"
}